heterochromatin formation [GO:0031507] (biological process) Subtypes: GO:0009048, regulatory ncRNA-mediated heterochromatin formation [GO:0031048], pericentric heterochromatin organization [GO:0140462], GO:0140718, constitutive heterochromatin formation [GO:0140719] Relationships: is a type of GO:0045814; has part heterochromatin boundary formation [GO:0033696] Definition: An epigenetic gene silencing mechanism in which chromatin is compacted into heterochromatin, resulting in a chromatin conformation refractory to transcription. This process starts with heterochromatin nucleation, its spreading, and ends with heterochromatin boundary formation. Regulation: regulated by regulation of heterochromatin formation [GO:0031445]; negatively regulated by negative regulation of heterochromatin formation [GO:0031452]; positively regulated by positive regulation of heterochromatin formation [GO:0031453] References: PMID:25192661, PMID:33827924 Also known as: TGS, heterochromatin maintenance, chromatin silencing, chromatin-mediated silencing, establishment of heterochromatin architecture, heterochromatin assembly, establishment of heterochromatin architecture involved in chromatin silencing at centromere outer repeat region, establishment of heterochromatin architecture involved in chromatin silencing at pericentric region, heterochromatin assembly involved in chromatin silencing at centromere outer repeat region, heterochromatin assembly involved in chromatin silencing at pericentric region, heterochromatin formation involved in chromatin silencing at centromere outer repeat region, heterochromatin formation involved in chromatin silencing at pericentric region, establishment of chromatin silencing, establishment of heterochromatic silencing, heterochromatic silencing, heterochromatin assembly involved in chromatin silencing, heterochromatin formation involved in chromatin silencing, transcriptional gene silencing